cyclic 2,3-diphosphoglycerate synthetase activity [GO:0036356] (molecular function) References: PMID:2226838, PMID:8320225, PMID:9811660 Sources: GOC:crds Note: This reaction is the intramolecular cyclization of 2,3-diphosphoglycerate to cyclic 2,3-diphosphoglycerate and is the second step in the biosynthesis of cyclic 2,3-diphosphoglycerate (cDPG). Definition: Catalysis of the reaction: 2,3-diphosphoglycerate (DPG) + ATP = cyclic 2,3-diphosphoglycerate (cDPG) + ADP + phosphate. Relationships: is a type of cyclase activity [GO:0009975]; is part of cyclic 2,3-bisphospho-D-glycerate biosynthetic process [GO:1901369] Also known as: CPGS activity, cDPGS activity